{
  "gene_name": "Signal transducer and activator of transcription 3",
  "term_label": "defense response",
  "gene": "UniProtKB:P40763",
  "term_id": "GO:0006952",
  "gene_symbol": "STAT3"
}